{
  "gene_symbol": "TMEM240",
  "gene_name": "Transmembrane protein 240",
  "term_id": "GO:0097060",
  "gene": "UniProtKB:Q5SV17",
  "term_label": "synaptic membrane"
}